{
  "term_label": "cortical actin cytoskeleton organization",
  "gene": "UniProtKB:Q15334",
  "gene_symbol": "LLGL1",
  "gene_name": "Lethal(2) giant larvae protein homolog 1",
  "term_id": "GO:0030866"
}